{
  "gene_symbol": "LRRC57",
  "gene_name": "Leucine-rich repeat-containing protein 57",
  "term_label": "Unknown biological process",
  "term_id": "UNKNOWN:0002",
  "gene": "UniProtKB:Q8N9N7"
}